{
  "gene_symbol": "KIF23",
  "gene_name": "Kinesin-like protein KIF23",
  "term_id": "GO:0005874",
  "gene": "UniProtKB:Q02241",
  "term_label": "microtubule"
}